{
  "gene_symbol": "PPP1R2P1",
  "gene_name": "Putative protein phosphatase inhibitor 2-like protein 1",
  "term_id": "GO:0035556",
  "gene": "UniProtKB:Q96PQ5",
  "term_label": "intracellular signal transduction"
}